{
  "gene_symbol": "COPZ2",
  "gene": "UniProtKB:Q9P299",
  "term_label": "Unknown molecular function",
  "term_id": "UNKNOWN:0001",
  "gene_name": "Coatomer subunit zeta-2"
}